regulation of cytokine production [GO:0001817] (biological process) Subtypes: negative regulation of cytokine production [GO:0001818], GO:0001819, GO:0002718, regulation of vascular endothelial growth factor production [GO:0010574], regulation of type I interferon production [GO:0032479], regulation of chemokine production [GO:0032642], regulation of connective tissue growth factor production [GO:0032643], GO:0032645, regulation of hepatocyte growth factor production [GO:0032646], regulation of type II interferon production [GO:0032649], regulation of interleukin-1 production [GO:0032652], regulation of interleukin-10 production [GO:0032653], GO:0032654, regulation of interleukin-12 production [GO:0032655], regulation of interleukin-13 production [GO:0032656], regulation of interleukin-15 production [GO:0032658], regulation of interleukin-16 production [GO:0032659], regulation of interleukin-17 production [GO:0032660], GO:0032661, regulation of interleukin-19 production [GO:0032662], regulation of interleukin-2 production [GO:0032663], regulation of interleukin-20 production [GO:0032664], regulation of interleukin-21 production [GO:0032665], GO:0032666, regulation of interleukin-23 production [GO:0032667], regulation of interleukin-24 production [GO:0032668], GO:0032669, regulation of interleukin-26 production [GO:0032670], regulation of interleukin-27 production [GO:0032671], regulation of interleukin-3 production [GO:0032672], regulation of interleukin-4 production [GO:0032673], GO:0032674, regulation of interleukin-6 production [GO:0032675], regulation of interleukin-7 production [GO:0032676], GO:0032677, GO:0032678, GO:0034344, regulation of interleukin-35 production [GO:0070754], GO:0071634, regulation of granzyme B production [GO:0071661], GO:0090270, GO:0090361, regulation of amphiregulin production [GO:0140731], regulation of interleukin-33 production [GO:0150127], regulation of interleukin-37 production [GO:0150136], regulation of interleukin-34 production [GO:0150157], regulation of interleukin-32 production [GO:0150189], regulation of cytokine production involved in inflammatory response [GO:1900015], regulation of glial cell-derived neurotrophic factor production [GO:1900166], regulation of macrophage colony-stimulating factor production [GO:1901256], GO:1903555, regulation of endothelin production [GO:1904470] Sources: GOC:add, ISBN:0781735149 Also known as: regulation of cytokine anabolism, regulation of cytokine biosynthesis, regulation of cytokine formation, regulation of cytokine synthesis, regulation of cytokine biosynthetic process, regulation of cytokine secretion Definition: Any process that modulates the frequency, rate, or extent of production of a cytokine. Relationships: is a type of GO:0010468; is a type of GO:0051239; RO_0002211 cytokine production [GO:0001816]